regulation of systemic arterial blood pressure by stress relaxation [GO:0003046] (biological process) Also known as: blood pressure regulation by stress relaxation Relationships: is a type of regulation of systemic arterial blood pressure by physical factors [GO:0003045]; is a type of negative regulation of systemic arterial blood pressure [GO:0003085] Definition: The intrinsic circulatory process resulting from stress relaxation that modulates the force with which blood travels through the systemic arterial circulatory system. Stress relaxation is the adaptation of vessels to a new size as a result of changes in pressure in storage areas such as veins, the liver, the spleen, and the lungs. Sources: GOC:mtg_cardio, ISBN:0721643949